{
  "term_label": "potassium ion import across plasma membrane",
  "gene": "UniProtKB:P48544",
  "term_id": "GO:1990573",
  "gene_symbol": "KCNJ5",
  "gene_name": "G protein-activated inward rectifier potassium channel 4"
}